{
  "gene_symbol": "COX16",
  "term_id": "UNKNOWN:0001",
  "gene_name": "Cytochrome c oxidase assembly protein COX16 homolog, mitochondrial",
  "gene": "UniProtKB:Q9P0S2",
  "term_label": "Unknown molecular function"
}